{
  "term_label": "cortical actin cytoskeleton organization",
  "term_id": "GO:0030866",
  "gene_symbol": "ROCK2",
  "gene_name": "Rho-associated protein kinase 2",
  "gene": "UniProtKB:O75116"
}